hydrogen peroxide mediated signaling pathway [GO:0071588] (biological process) References: PMID:17043891 Sources: GOC:mah Also known as: H2O2 mediated signaling pathway, hydrogen peroxide mediated signalling pathway Definition: The series of molecular signals mediated by the detection of hydrogen peroxide (H2O2). Relationships: is_a signal transduction [GO:0007165]